(-)-borneol dehydrogenase activity [GO:0047503] (molecular function) Definition: Catalysis of the reaction: (-)-borneol + NAD+ = (1S,4S)-camphor + H+ + NADH. Sources: EC:1.1.1.227, RHEA:22128 Also known as: (-)-borneol:NAD+ oxidoreductase activity Relationships: is a type of oxidoreductase activity, acting on the CH-OH group of donors, NAD or NADP as acceptor [GO:0016616]